{
  "term_label": "nucleus",
  "gene": "UniProtKB:Q9UIK4",
  "gene_symbol": "DAPK2",
  "term_id": "GO:0005634",
  "gene_name": "Death-associated protein kinase 2"
}